{
  "term_id": "GO:0005730",
  "gene": "UniProtKB:Q9Y421",
  "term_label": "nucleolus",
  "gene_symbol": "FAM32A",
  "gene_name": "Protein FAM32A"
}